2-hydroxyacyl-CoA lyase activity [GO:0106359] (molecular function) Definition: Catalysis of the reaction: a 2-hydroxy fatty acyl-CoA = a fatty aldehyde + formyl-CoA. The reaction acts on 2-hydroxy-3-methyl-branched fatty acyl-CoA and 2-hydroxy-long-chain fatty acyl-CoA. References: PMID:21708296, PMID:28289220 Sources: EC:4.1.2.63 Relationships: is a type of aldehyde-lyase activity [GO:0016832] Subtypes: 2-hydroxyphytanoyl-CoA lyase activity [GO:0106376]